{
  "term_id": "GO:0046854",
  "gene_name": "Inositol-trisphosphate 3-kinase C",
  "term_label": "phosphatidylinositol phosphate biosynthetic process",
  "gene": "UniProtKB:Q96DU7",
  "gene_symbol": "ITPKC"
}